symbiont-mediated perturbation of host B-cell mediated immune response [GO:0052154] (biological process) Also known as: modulation by organism of B-cell mediated immune response of other organism involved in symbiotic interaction, modulation by symbiont of host B-cell mediated immune response, perturbation of host B-cell mediated immune response, regulation by organism of host B-cell mediated immune response, symbiont-mediated perturbation of host humoral immune response Sources: GOC:mtg_pamgo_17jul06 Definition: A process in which a symbiont alters or subverts the B-cell mediated immune response of the host organism. The host is defined as the larger of the organisms involved in a symbiotic interaction. Relationships: is_a GO:0052553